{
  "gene_name": "Immunoglobulin subtype domain-containing protein",
  "gene": "UniProtKB:A0A5F9ZH88",
  "term_label": "transmembrane signaling receptor activity",
  "term_id": "GO:0004888",
  "gene_symbol": "A0A5F9ZH88"
}